{
  "gene": "UniProtKB:A6NM10",
  "term_label": "Unknown biological process",
  "gene_name": "Aquaporin-12B",
  "term_id": "UNKNOWN:0002",
  "gene_symbol": "AQP12B"
}